{
  "gene_symbol": "EBLN1",
  "gene_name": "Endogenous Bornavirus-like nucleoprotein 1",
  "term_label": "Unknown molecular function",
  "gene": "UniProtKB:P0CF75",
  "term_id": "UNKNOWN:0001"
}